{
  "gene": "UniProtKB:Q9Y6A4",
  "term_label": "motile cilium",
  "gene_name": "Cilia- and flagella-associated protein 20",
  "gene_symbol": "CFAP20",
  "term_id": "GO:0031514"
}